{
  "term_label": "positive regulation of canonical NF-kappaB signal transduction",
  "gene_symbol": "TICAM1",
  "gene": "UniProtKB:Q8IUC6",
  "term_id": "GO:0043123",
  "gene_name": "TIR domain-containing adapter molecule 1"
}